glycine binding [GO:0016594] (MF) Sources: GOC:ai Also known as: Gly binding, aminoacetic acid binding, aminoethanoic acid binding Relationships: is a type of amino acid binding [GO:0016597]; is a type of carboxylic acid binding [GO:0031406]; is a type of cation binding [GO:0043169] Definition: Binding to glycine, aminoethanoic acid.